{
  "gene_symbol": "GNAI3",
  "term_label": "G protein-coupled receptor binding",
  "gene": "UniProtKB:P08754",
  "gene_name": "Guanine nucleotide-binding protein G(i) subunit alpha-3",
  "term_id": "GO:0001664"
}